{
  "gene": "UniProtKB:P09012",
  "term_label": "U1 snRNA binding",
  "gene_symbol": "SNRPA",
  "term_id": "GO:0030619",
  "gene_name": "U1 small nuclear ribonucleoprotein A"
}